2-deoxyribose 1-phosphate catabolic process [GO:0006018] (biological process) Definition: The chemical reactions and pathways resulting in the breakdown of deoxyribose 1-phosphate, the phosphorylated sugar 1-phospho-2-deoxyribose. Relationships: is a type of deoxyribose phosphate catabolic process [GO:0046386] Sources: GOC:ai Also known as: 2-deoxyribose 1-phosphate breakdown, 2-deoxyribose 1-phosphate catabolism, 2-deoxyribose 1-phosphate degradation, deoxyribose 1-phosphate catabolic process